{
  "gene_symbol": "TBR1",
  "term_label": "nucleus",
  "gene_name": "T-box brain protein 1",
  "term_id": "GO:0005634",
  "gene": "UniProtKB:Q16650"
}